negative regulation of retinoic acid biosynthetic process [GO:1900053] (biological process) Definition: Any process that stops, prevents or reduces the frequency, rate or extent of retinoic acid biosynthetic process. Also known as: down regulation of retinoic acid anabolic process, down-regulation of retinoic acid anabolic process, downregulation of retinoic acid anabolic process, inhibition of retinoic acid anabolic process, negative regulation of retinoic acid anabolic process, down regulation of retinoic acid biosynthetic process, down-regulation of retinoic acid biosynthetic process, downregulation of retinoic acid biosynthetic process, inhibition of retinoic acid biosynthetic process Sources: GOC:TermGenie, GOC:yaf Relationships: is a type of GO:0032351; is a type of GO:0045827; is a type of negative regulation of vitamin metabolic process [GO:0046137]; is a type of GO:0051055; is a type of regulation of retinoic acid biosynthetic process [GO:1900052]; negatively regulates retinoic acid biosynthetic process [GO:0002138]